{
  "term_id": "GO:0005829",
  "term_label": "cytosol",
  "gene_symbol": "IRS1",
  "gene": "UniProtKB:P35568",
  "gene_name": "Insulin receptor substrate 1"
}